{
  "term_label": "regulation of transcription by RNA polymerase II",
  "gene_name": "Zinc finger protein 786",
  "gene": "UniProtKB:Q8N393",
  "term_id": "GO:0006357",
  "gene_symbol": "ZNF786"
}